{
  "term_id": "GO:0006357",
  "gene": "UniProtKB:Q8IUR6",
  "term_label": "regulation of transcription by RNA polymerase II",
  "gene_symbol": "CREBRF",
  "gene_name": "CREB3 regulatory factor"
}